pyridoxal transmembrane transport [GO:1903090] (biological process) References: PMID:15701794 Sources: GOC:TermGenie, GO_REF:0000069 Definition: The process in which pyridoxal is transported across a membrane. Subtypes: GO:0140204 Relationships: is a type of pyridoxal transport [GO:0031920]; is a type of vitamin transmembrane transport [GO:0035461]